{
  "term_id": "GO:0000981",
  "gene": "UniProtKB:P12980",
  "gene_symbol": "LYL1",
  "gene_name": "Protein lyl-1",
  "term_label": "DNA-binding transcription factor activity, RNA polymerase II-specific"
}